{
  "term_label": "Unknown cellular component",
  "gene": "UniProtKB:Q6L8H4",
  "term_id": "UNKNOWN:0003",
  "gene_symbol": "KRTAP5-1",
  "gene_name": "Keratin-associated protein 5-1"
}